{
  "term_id": "GO:0005634",
  "gene": "UniProtKB:Q9H9J2",
  "term_label": "nucleus",
  "gene_symbol": "MRPL44",
  "gene_name": "Large ribosomal subunit protein mL44"
}